{
  "gene_name": "E3 ubiquitin-protein ligase RNF43",
  "gene": "UniProtKB:Q68DV7",
  "term_id": "GO:0005886",
  "gene_symbol": "RNF43",
  "term_label": "plasma membrane"
}